{
  "gene_name": "Forkhead box protein M1",
  "gene": "UniProtKB:Q08050",
  "gene_symbol": "FOXM1",
  "term_id": "GO:0006355",
  "term_label": "regulation of DNA-templated transcription"
}